{
  "gene_name": "DnaJ homolog subfamily A member 2",
  "gene": "UniProtKB:O60884",
  "term_label": "cytosol",
  "gene_symbol": "DNAJA2",
  "term_id": "GO:0005829"
}